TTP catabolic process [GO:0046047] (biological process) Also known as: TTP breakdown, TTP catabolism, TTP degradation, TTP hydrolysis Definition: The chemical reactions and pathways resulting in the breakdown of TTP, ribosylthymine triphosphate. Relationships: is_a GO:0009210; is a type of pyrimidine ribonucleotide catabolic process [GO:0009222]; is a type of GO:0046046 Sources: GOC:go_curators